{
  "term_id": "UNKNOWN:0001",
  "gene_name": "GATOR complex protein MIOS",
  "term_label": "Unknown molecular function",
  "gene_symbol": "MIOS",
  "gene": "UniProtKB:Q9NXC5"
}